{
  "gene_symbol": "DPPA3",
  "term_id": "GO:0044726",
  "gene_name": "Developmental pluripotency-associated protein 3",
  "term_label": "epigenetic programing of female pronucleus",
  "gene": "UniProtKB:Q6W0C5"
}